{
  "gene_symbol": "KCNQ2",
  "term_id": "GO:0001508",
  "gene_name": "Potassium voltage-gated channel subfamily KQT member 2",
  "term_label": "action potential",
  "gene": "UniProtKB:O43526"
}